cellular response to beta-carotene [GO:1905388] (biological process) Definition: Any process that results in a change in state or activity of a cell (in terms of movement, secretion, enzyme production, gene expression, etc.) as a result of a beta-carotene stimulus. References: PMID:16771696 Sources: GOC:TermGenie, GO_REF:0000071 Relationships: is_a cellular response to lipid [GO:0071396]; is_a response to beta-carotene [GO:1905387] Also known as: cellular response to beta,beta-carotene